long-chain fatty acid biosynthetic process [GO:0042759] (biological process) Subtypes: jasmonic acid biosynthetic process [GO:0009695], hepoxilin biosynthetic process [GO:0051122], leukotriene B4 biosynthetic process [GO:0097251], resolvin biosynthetic process [GO:0106295], palmitic acid biosynthetic process [GO:1900535], leukotriene A4 biosynthetic process [GO:1901753], GO:1902609, lipoxin A4 biosynthetic process [GO:2001303], GO:2001306 References: PMID:18390550 Definition: The chemical reactions and pathways resulting in the formation of a long-chain fatty acid. A long-chain fatty acid has an aliphatic tail containing 13 to 22 carbons. Relationships: is a type of long-chain fatty acid metabolic process [GO:0001676]; is a type of fatty acid biosynthetic process [GO:0006633] Also known as: long-chain fatty acid anabolism, long-chain fatty acid biosynthesis, long-chain fatty acid formation, long-chain fatty acid synthesis Note: While there is not universal consensus on the lengths of short-, medium-, long- and very-long-chain fatty acids, the GO uses the definitions in ChEBI (see CHEBI:26666, CHEBI:59554, CHEBI:15904 and CHEBI:27283).